positive regulation of metalloendopeptidase activity [GO:1904685] (biological process) Also known as: up regulation of metalloendopeptidase activity, up-regulation of metalloendopeptidase activity, upregulation of metalloendopeptidase activity, activation of metalloendopeptidase activity, activation of metalloendoprotease activity, activation of metalloendoproteinase activity, positive regulation of metalloendoprotease activity, positive regulation of metalloendoproteinase activity, up regulation of metalloendoprotease activity, up regulation of metalloendoproteinase activity, up-regulation of metalloendoprotease activity, up-regulation of metalloendoproteinase activity, upregulation of metalloendoprotease activity, upregulation of metalloendoproteinase activity References: PMID:18591254 Sources: GOC:BHF, GOC:BHF_miRNA, GOC:TermGenie, GOC:rph, GO_REF:0000059 Relationships: is a type of positive regulation of endopeptidase activity [GO:0010950]; is a type of positive regulation of metallopeptidase activity [GO:1905050]; positively regulates metalloendopeptidase activity [GO:0004222] Definition: Any process that activates or increases the frequency, rate or extent of metalloendopeptidase activity.